{
  "gene_symbol": "VSIG4",
  "term_id": "GO:0001851",
  "gene": "UniProtKB:Q9Y279",
  "gene_name": "V-set and immunoglobulin domain-containing protein 4",
  "term_label": "complement component C3b binding"
}